non-canonical inflammasome complex assembly [GO:0160075] (biological process) Definition: The aggregation, arrangement and bonding together of a set of components to form a non-canonical inflammasome complex. Relationships: is a type of protein-containing complex assembly [GO:0065003] Regulation: negatively regulated by negative regulation of non-canonical inflammasome complex assembly [GO:0160076] References: PMID:27291964